negative regulation of chromosome attachment to the nuclear envelope [GO:0120265] (biological process) Relationships: is_a negative regulation of cell cycle process [GO:0010948]; is a type of GO:0120264; negatively regulates chromosome attachment to the nuclear envelope [GO:0097240] Also known as: down regulation of chromosome attachment to the nuclear envelope, down-regulation of chromosome attachment to the nuclear envelope, downregulation of chromosome attachment to the nuclear envelope, inhibition of chromosome attachment to the nuclear envelope Definition: Any process that stops, prevents, or reduces the frequency, rate or extent of the chromosome attachment to the nuclear envelope. Sources: GOC:krc